{
  "gene_symbol": "ELOVL3",
  "gene_name": "Elongation of very long chain fatty acids protein 3",
  "term_label": "endoplasmic reticulum membrane",
  "gene": "UniProtKB:Q9HB03",
  "term_id": "GO:0005789"
}